{
  "gene_name": "Interferon alpha-16",
  "gene": "UniProtKB:P05015",
  "gene_symbol": "IFNA16",
  "term_label": "adaptive immune response",
  "term_id": "GO:0002250"
}